regulation of phosphatidylcholine catabolic process [GO:0010899] (biological process) Relationships: is a type of regulation of phospholipid catabolic process [GO:0060696]; is a type of GO:0150172; regulates phosphatidylcholine catabolic process [GO:0034638] Subtypes: negative regulation of phosphatidylcholine catabolic process [GO:0010900] Definition: Any process that modulates the rate, frequency or extent of phosphatidylcholine catabolism. Phosphatidylcholine catabolic processes are the chemical reactions and pathways resulting in the breakdown of phosphatidylcholines, any of a class of glycerophospholipids in which the phosphatidyl group is esterified to the hydroxyl group of choline. Sources: GOC:BHF, GOC:tb